regulation of diacylglycerol biosynthetic process [GO:1900480] (biological process) Definition: Any process that modulates the frequency, rate or extent of diacylglycerol biosynthetic process. Also known as: regulation of diacylglycerol anabolism, regulation of diacylglycerol biosynthesis, regulation of diacylglycerol formation, regulation of diacylglycerol synthesis Subtypes: GO:1900481, positive regulation of diacylglycerol biosynthetic process [GO:1900482] Relationships: is a type of regulation of lipid biosynthetic process [GO:0046890]; regulates GO:0006651 Sources: GOC:TermGenie